{
  "term_label": "Unknown molecular function",
  "term_id": "UNKNOWN:0001",
  "gene_name": "COMM domain-containing protein 1",
  "gene_symbol": "COMMD1",
  "gene": "UniProtKB:Q8N668"
}